negative regulation of translational initiation [GO:0045947] (biological process) Sources: GOC:go_curators Also known as: down regulation of translational initiation, down-regulation of translational initiation, downregulation of translational initiation, inhibition of translational initiation Subtypes: negative regulation of translational initiation in response to stress [GO:0032057], negative regulation of translational initiation by iron [GO:0045993], negative regulation of mitochondrial translational initiation [GO:0070133], negative regulation of formation of translation initiation ternary complex [GO:1901191], negative regulation of cytoplasmic translational initiation [GO:1904689] Relationships: is a type of regulation of translational initiation [GO:0006446]; is a type of negative regulation of translation [GO:0017148]; negatively regulates translational initiation [GO:0006413] Definition: Any process that stops, prevents, or reduces the frequency, rate or extent of translational initiation.